{
  "term_id": "UNKNOWN:0001",
  "gene_symbol": "KNCN",
  "term_label": "Unknown molecular function",
  "gene_name": "Kinocilin",
  "gene": "UniProtKB:A6PVL3"
}